{
  "term_label": "mRNA N6-methyladenosine dioxygenase activity",
  "gene_name": "Alpha-ketoglutarate-dependent dioxygenase FTO",
  "term_id": "GO:1990931",
  "gene": "UniProtKB:Q9C0B1",
  "gene_symbol": "FTO"
}